cellular response to trichodermin [GO:0072744] (biological process) Definition: Any process that results in a change in state or activity of a cell (in terms of movement, secretion, enzyme production, gene expression, etc.) as a result of a trichodermin stimulus. Sources: GOC:mah Relationships: is a type of cellular response to ether [GO:0071362]; is a type of response to trichodermin [GO:1901324]